{
  "gene_name": "Zinc finger protein 322",
  "term_id": "GO:0006357",
  "gene_symbol": "ZNF322",
  "term_label": "regulation of transcription by RNA polymerase II",
  "gene": "UniProtKB:Q6U7Q0"
}